{
  "gene_symbol": "SMYD3",
  "gene": "UniProtKB:Q9H7B4",
  "term_label": "heart development",
  "term_id": "GO:0007507",
  "gene_name": "Histone-lysine N-methyltransferase SMYD3"
}